regulation of phosphatidylserine biosynthetic process [GO:1900468] (biological process) Definition: Any process that modulates the frequency, rate or extent of phosphatidylserine biosynthetic process. References: PMID:8056324, PMID:8614637 Sources: GOC:TermGenie, GOC:dgf Also known as: regulation of phosphatidylserine anabolism, regulation of phosphatidylserine biosynthesis, regulation of phosphatidylserine formation, regulation of phosphatidylserine synthesis Relationships: is a type of regulation of phospholipid biosynthetic process [GO:0071071]; regulates phosphatidylserine biosynthetic process [GO:0006659] Subtypes: negative regulation of phosphatidylserine biosynthetic process [GO:1900469], positive regulation of phosphatidylserine biosynthetic process [GO:1900470]